{
  "term_label": "nuclear receptor activity",
  "term_id": "GO:0004879",
  "gene_symbol": "VDR",
  "gene_name": "Vitamin D3 receptor",
  "gene": "UniProtKB:P11473"
}